venom-mediated perturbation of transmission of nerve impulse [GO:0044487] (biological process) Definition: A process in which an organism alters or subverts the transmission of a nerve impulse in another organism via the action of a venom. Sources: GOC:fj, GOC:jl Relationships: is a type of GO:0140136 Also known as: envenomation resulting in modulation of conduction of nerve impulse in other organism, envenomation resulting in modulation of transmission of nerve impulse in another organism, envenomation resulting in modulation of transmission of nerve impulse in other organism